fruit dehiscence [GO:0010047] (biological process) Definition: The process leading to the spontaneous opening of the fruit permitting the escape of seeds. Sources: GOC:tb, ISBN:0471245208 Relationships: is a type of dehiscence [GO:0009900]